{
  "term_id": "UNKNOWN:0002",
  "gene": "UniProtKB:A0A1B0GUV8",
  "gene_name": "Lipocalin_cytosolic fatty-acid binding domain-containing protein",
  "gene_symbol": "LOC102723971",
  "term_label": "Unknown biological process"
}